{
  "term_id": "GO:0007411",
  "gene_name": "Ena_VASP-like protein",
  "term_label": "axon guidance",
  "gene": "UniProtKB:Q9UI08",
  "gene_symbol": "EVL"
}